arginine racemase activity [GO:0047679] (molecular function) Sources: EC:5.1.1.9, MetaCyc:ARGININE-RACEMASE-RXN Relationships: is a type of amino-acid racemase activity [GO:0047661] Definition: Catalysis of the reaction: L-arginine = D-arginine.